positive regulation of type IV pilus biogenesis [GO:1903658] (biological process) Definition: Any process that activates or increases the frequency, rate or extent of type IV pilus biogenesis. Relationships: is a type of positive regulation of cell projection organization [GO:0031346]; is a type of regulation of type IV pilus biogenesis [GO:1903656]; positively regulates type IV pilus assembly [GO:0043683] Also known as: positive regulation of TFP biogenesis, positive regulation of type 4 pilus biogenesis, positive regulation of type IV fimbria assembly, positive regulation of type IV fimbria biogenesis, positive regulation of type IV fimbriae assembly, positive regulation of type IV fimbriae biogenesis, positive regulation of type IV fimbrial assembly, positive regulation of type IV fimbrial biogenesis, positive regulation of type IV fimbrium assembly, positive regulation of type IV fimbrium biogenesis, positive regulation of type IV pilus biosynthesis, up regulation of TFP biogenesis, up regulation of type 4 pilus biogenesis, up regulation of type IV fimbria assembly, up regulation of type IV fimbria biogenesis, up regulation of type IV fimbriae assembly, up regulation of type IV fimbriae biogenesis, up regulation of type IV fimbrial assembly, up regulation of type IV fimbrial biogenesis, up regulation of type IV fimbrium assembly, up regulation of type IV fimbrium biogenesis, up regulation of type IV pilus biogenesis, up regulation of type IV pilus biosynthesis, up-regulation of TFP biogenesis, up-regulation of type 4 pilus biogenesis, up-regulation of type IV fimbria assembly, up-regulation of type IV fimbria biogenesis, up-regulation of type IV fimbriae assembly, up-regulation of type IV fimbriae biogenesis, up-regulation of type IV fimbrial assembly, up-regulation of type IV fimbrial biogenesis, up-regulation of type IV fimbrium assembly, up-regulation of type IV fimbrium biogenesis, up-regulation of type IV pilus biogenesis, up-regulation of type IV pilus biosynthesis, upregulation of TFP biogenesis, upregulation of type 4 pilus biogenesis, upregulation of type IV fimbria assembly, upregulation of type IV fimbria biogenesis, upregulation of type IV fimbriae assembly, upregulation of type IV fimbriae biogenesis, upregulation of type IV fimbrial assembly, upregulation of type IV fimbrial biogenesis, upregulation of type IV fimbrium assembly, upregulation of type IV fimbrium biogenesis, upregulation of type IV pilus biogenesis, upregulation of type IV pilus biosynthesis, activation of TFP biogenesis, activation of type 4 pilus biogenesis, activation of type IV fimbria assembly, activation of type IV fimbria biogenesis, activation of type IV fimbriae assembly, activation of type IV fimbriae biogenesis, activation of type IV fimbrial assembly, activation of type IV fimbrial biogenesis, activation of type IV fimbrium assembly, activation of type IV fimbrium biogenesis, activation of type IV pilus biogenesis, activation of type IV pilus biosynthesis References: PMID:25049409 Sources: GOC:TermGenie, GO_REF:0000058